{
  "term_label": "phototransduction, visible light",
  "gene": "UniProtKB:A8MTJ3",
  "gene_name": "Guanine nucleotide-binding protein G(t) subunit alpha-3",
  "gene_symbol": "GNAT3",
  "term_id": "GO:0007603"
}